acquisition of seed longevity [GO:0140547] (BP) Relationships: is a type of multicellular organismal process [GO:0032501]; is part of seed development [GO:0048316] Definition: The acquisition of seed longevity is the ordered series of events during seed development, that prevent embryo deterioration and ROS damage and thus contribute to seed viability over time or in response to adverse environmental conditions. These events include protective (e.g. production of glassy cytoplasm ) and repair (e.g. oxidative stress responses) processes. References: PMID:26637538